{
  "gene": "UniProtKB:Q96DZ1",
  "term_id": "UNKNOWN:0001",
  "gene_symbol": "ERLEC1",
  "gene_name": "Endoplasmic reticulum lectin 1",
  "term_label": "Unknown molecular function"
}